{
  "gene_name": "U3 small nucleolar RNA-associated protein 6 homolog",
  "gene": "UniProtKB:Q9NYH9",
  "term_label": "Pwp2p-containing subcomplex of 90S preribosome",
  "gene_symbol": "UTP6",
  "term_id": "GO:0034388"
}